{
  "gene": "UniProtKB:A0A1B0GUA9",
  "term_label": "Unknown cellular component",
  "term_id": "UNKNOWN:0003",
  "gene_symbol": "C13orf46",
  "gene_name": "Uncharacterized protein C13orf46"
}